{
  "gene_name": "Zinc finger protein 737",
  "gene_symbol": "ZNF737",
  "gene": "UniProtKB:O75373",
  "term_id": "UNKNOWN:0003",
  "term_label": "Unknown cellular component"
}